{
  "gene": "UniProtKB:Q9Y676",
  "gene_symbol": "MRPS18B",
  "term_id": "UNKNOWN:0001",
  "term_label": "Unknown molecular function",
  "gene_name": "Small ribosomal subunit protein mS40"
}